{
  "term_id": "UNKNOWN:0003",
  "gene_name": "T cell receptor gamma constant 2",
  "gene": "UniProtKB:P03986",
  "term_label": "Unknown cellular component",
  "gene_symbol": "TRGC2"
}